{
  "gene": "UniProtKB:Q5SQN1",
  "gene_name": "Synaptosomal-associated protein 47",
  "term_id": "GO:0019905",
  "term_label": "syntaxin binding",
  "gene_symbol": "SNAP47"
}